{
  "term_label": "nuclear import signal receptor activity",
  "term_id": "GO:0061608",
  "gene_name": "Importin subunit alpha-3",
  "gene_symbol": "KPNA4",
  "gene": "UniProtKB:O00629"
}